{
  "gene_symbol": "POM121L12",
  "term_label": "Unknown molecular function",
  "gene_name": "POM121-like protein 12",
  "gene": "UniProtKB:Q8N7R1",
  "term_id": "UNKNOWN:0001"
}